metanephric capsule formation [GO:0072266] (biological process) Relationships: is a type of renal capsule formation [GO:0072129]; is part of metanephric capsule morphogenesis [GO:0072265] Definition: The developmental process pertaining to the initial formation of a metanephric capsule from unspecified parts. The metanephric capsule is the tough fibrous layer surrounding the metanephros, covered in a thick layer of perinephric adipose tissue. It provides some protection from trauma and damage. Sources: GOC:mtg_kidney_jan10